endosomal transport [GO:0016197] (biological process) Relationships: is a type of vesicle-mediated transport [GO:0016192]; is a type of intracellular transport [GO:0046907] Subtypes: GO:0032456, GO:0032509, retrograde transport, endosome to Golgi [GO:0042147], trans-Golgi network to recycling endosome transport [GO:0044795], GO:0098927, GO:0099532 Definition: The directed movement of substances mediated by an endosome, a membrane-bounded organelle that carries materials enclosed in the lumen or located in the endosomal membrane. Sources: ISBN:0198506732 Also known as: endosome localisation, endosome localization, endosome transport